Arp2/3 complex binding [GO:0071933] (MF) Relationships: is a type of protein-containing complex binding [GO:0044877] Sources: GOC:mah Definition: Binding to an Arp2/3 complex, a protein complex that contains two actin-related proteins, Arp2 and Arp3, and five novel proteins (ARPC1-5).